{
  "term_label": "Unknown biological process",
  "gene_symbol": "SETD6",
  "term_id": "UNKNOWN:0002",
  "gene": "UniProtKB:Q8TBK2",
  "gene_name": "N-lysine methyltransferase SETD6"
}